iridophore differentiation [GO:0050935] (BP) Regulation: RO_0002211 by regulation of iridophore differentiation [GO:0050937]; RO_0002212 by negative regulation of iridophore differentiation [GO:0050943]; positively regulated by positive regulation of iridophore differentiation [GO:0050945] Relationships: is a type of GO:0050931 References: PMID:11858836 Sources: GOC:jid, GOC:mh Definition: The process in which a relatively unspecialized cell acquires the specialized features of an iridophore. Iridophores are pigment cells derived from the neural crest. They contain guanidine or other purine crystals deposited in stacks called reflecting platets or iridisomes. This gives them a silver, gold, or iridescent appearance. Also known as: iridophore cell differentiation